{
  "gene": "UniProtKB:Q9Y234",
  "gene_symbol": "LIPT1",
  "term_id": "GO:0005737",
  "gene_name": "Lipoyltransferase 1, mitochondrial",
  "term_label": "cytoplasm"
}